nitric-oxide synthase regulator activity [GO:0030235] (molecular function) Definition: Binds to and modulates the activity of nitric oxide synthase. Also known as: nitric oxide synthase regulator activity Sources: GOC:mah Relationships: is a type of enzyme regulator activity [GO:0030234]; has part nitric-oxide synthase binding [GO:0050998]; regulates nitric-oxide synthase activity [GO:0004517] Note: See also 'regulation of nitric-oxide synthase activity ; GO:0050999'. Subtypes: nitric-oxide synthase inhibitor activity [GO:0036487]